{
  "gene_name": "DNA dC-dU-editing enzyme APOBEC-3G",
  "term_label": "cytidine to uridine editing",
  "gene_symbol": "APOBEC3G",
  "gene": "UniProtKB:Q9HC16",
  "term_id": "GO:0016554"
}